{
  "gene": "UniProtKB:Q8NFW5",
  "gene_symbol": "DMBX1",
  "term_id": "GO:0000977",
  "term_label": "RNA polymerase II transcription regulatory region sequence-specific DNA binding",
  "gene_name": "Diencephalon_mesencephalon homeobox protein 1"
}